steroid N-acetylglucosaminyltransferase activity [GO:0047261] (molecular function) Also known as: UDP-N-acetyl-D-glucosamine:estradiol-17alpha-3-D-glucuronoside 17alpha-N-acetylglucosaminyltransferase activity, hydroxy steroid acetylglucosaminyltransferase activity, steroid acetylglucosaminyltransferase activity, uridine diphosphoacetylglucosamine-steroid acetylglucosaminyltransferase activity Relationships: is a type of GO:0008375 Sources: EC:2.4.1.39, RHEA:14153 Definition: Catalysis of the reaction: estradiol-17alpha 3-D-glucuronoside + UDP-N-acetyl-alpha-D-glucosamine = 17alpha-(N-acetyl-D-glucosaminyl)-estradiol 3-D-glucuronoside + H+ + UDP.